regulation of granulocyte macrophage colony-stimulating factor production [GO:0032645] (biological process) Definition: Any process that modulates the frequency, rate, or extent of granulocyte macrophage colony-stimulating factor production. Sources: GOC:mah Also known as: regulation of GM-CSF production, regulation of granulocyte macrophage colony stimulating factor production, regulation of granulocyte macrophage colony-stimulating factor biosynthetic process Relationships: is a type of regulation of cytokine production [GO:0001817]; is_a regulation of protein metabolic process [GO:0051246]; regulates granulocyte macrophage colony-stimulating factor production [GO:0032604] Subtypes: GO:0032685, positive regulation of granulocyte macrophage colony-stimulating factor production [GO:0032725]